{
  "term_label": "Unknown cellular component",
  "term_id": "UNKNOWN:0003",
  "gene": "UniProtKB:Q4LDG9",
  "gene_name": "Dynein axonemal light chain 1",
  "gene_symbol": "DNAL1"
}